limb granular cell fate specification [GO:0060893] (biological process) Definition: The process in which a cell becomes capable of differentiating autonomously into an limb granular cell in an environment that is neutral with respect to the developmental pathway; upon specification, the cell fate can be reversed. Sources: GOC:dph, GOC:sdb_2009, GOC:tb Relationships: is a type of GO:0009957; is a type of cell fate specification involved in pattern specification [GO:0060573]; is part of limb epidermis stratification [GO:0060888]; BFO_0000050 limb granular cell differentiation [GO:0060891]